{
  "term_label": "nucleus",
  "gene_symbol": "EID3",
  "term_id": "GO:0005634",
  "gene_name": "EP300-interacting inhibitor of differentiation 3",
  "gene": "UniProtKB:Q8N140"
}